latency-replication decision [GO:0098689] (biological process) Also known as: Latency-replication switch, lytic switch, proviral induction, proviral switch, reactivation of latent virus, prophage induction Relationships: is a type of GO:0016032; regulates release from viral latency [GO:0019046] Definition: The process by which a virus switches on its replication cycle in an infected cell. The process is typically controlled by a genetic switch controlled by environmental factors such as cell type, cell shape, the availability of nutrients, superinfection or exposure of infected cells to UV or various chemical stimuli. References: PMID:19416825, PMID:24339346 Sources: VZ:3964